{
  "term_id": "GO:0045727",
  "term_label": "positive regulation of translation",
  "gene": "UniProtKB:Q92615",
  "gene_name": "La-related protein 4B",
  "gene_symbol": "LARP4B"
}